{
  "term_label": "T cell receptor signaling pathway",
  "gene_name": "Butyrophilin-like protein 2",
  "term_id": "GO:0050852",
  "gene": "UniProtKB:Q9UIR0",
  "gene_symbol": "BTNL2"
}